cytosolic tRNA wobble base thiouridylase complex [GO:0002144] (cellular component) References: PMID:17062623, PMID:18391219 Definition: A complex of two proteins involved in the thiolation of uridine 34 (U34) of tRNAs decoding two-family box triplets. Relationships: is a type of intracellular protein-containing complex [GO:0140535]; is a type of GO:1990228 Also known as: tRNA thiouridylase, Ctu1-Ctu2 complex